{
  "gene": "UniProtKB:Q9ULW6",
  "gene_symbol": "NAP1L2",
  "gene_name": "Nucleosome assembly protein 1-like 2",
  "term_label": "histone binding",
  "term_id": "GO:0042393"
}